{
  "gene": "UniProtKB:Q8NCW5",
  "term_label": "Unknown biological process",
  "gene_name": "NAD(P)H-hydrate epimerase",
  "term_id": "UNKNOWN:0002",
  "gene_symbol": "NAXE"
}